{
  "gene_name": "Mixed lineage kinase domain-like protein",
  "gene_symbol": "MLKL",
  "term_label": "cytoplasm",
  "term_id": "GO:0005737",
  "gene": "UniProtKB:Q8NB16"
}